negative regulation of phialide development [GO:0070806] (biological process) Relationships: is a type of GO:0010721; is a type of negative regulation of conidiophore development [GO:0070794]; is a type of GO:0070805; negatively regulates phialide development [GO:0070790] Definition: Any process that stops, prevents, or reduces the frequency, rate or extent of phialide development, a process that leads to the formation of phialides. Phialides are specialized cells that bud from the ends of metulae on the conidiophore tip. Sources: GOC:mah